{
  "gene": "UniProtKB:Q96DM3",
  "term_id": "GO:0031902",
  "term_label": "late endosome membrane",
  "gene_name": "Regulator of MON1-CCZ1 complex",
  "gene_symbol": "RMC1"
}